{
  "gene": "UniProtKB:Q7Z7H5",
  "gene_symbol": "TMED4",
  "gene_name": "Transmembrane emp24 domain-containing protein 4",
  "term_label": "COPII-coated ER to Golgi transport vesicle",
  "term_id": "GO:0030134"
}